{
  "term_label": "cilium assembly",
  "gene_name": "Centriole and centriolar satellite protein OFD1",
  "term_id": "GO:0060271",
  "gene": "UniProtKB:O75665",
  "gene_symbol": "OFD1"
}